{
  "term_id": "GO:0002116",
  "gene": "UniProtKB:Q9Y4D7",
  "term_label": "semaphorin receptor complex",
  "gene_symbol": "PLXND1",
  "gene_name": "Plexin-D1"
}